{
  "gene": "UniProtKB:P41247",
  "term_label": "membrane",
  "gene_symbol": "PNPLA4",
  "gene_name": "Patatin-like phospholipase domain-containing protein 4",
  "term_id": "GO:0016020"
}